{
  "gene_name": "Splicing factor 3B subunit 6",
  "term_id": "UNKNOWN:0002",
  "gene": "UniProtKB:Q9Y3B4",
  "term_label": "Unknown biological process",
  "gene_symbol": "SF3B6"
}